{
  "gene": "UniProtKB:A0A0B4J275",
  "gene_symbol": "TRAV17",
  "term_label": "Unknown cellular component",
  "term_id": "UNKNOWN:0003",
  "gene_name": "T cell receptor alpha variable 17"
}